{
  "term_id": "UNKNOWN:0003",
  "gene": "UniProtKB:A0A140TA67",
  "gene_symbol": "KRTAP9-6",
  "gene_name": "Keratin-associated protein 9-6",
  "term_label": "Unknown cellular component"
}